{
  "term_id": "UNKNOWN:0001",
  "gene_name": "Putative protein BCL8",
  "term_label": "Unknown molecular function",
  "gene": "UniProtKB:P0C6P0",
  "gene_symbol": "NBEAP1"
}